{
  "gene": "UniProtKB:P15516",
  "gene_name": "Histatin-3",
  "term_label": "extracellular space",
  "term_id": "GO:0005615",
  "gene_symbol": "HTN3"
}